fructose 5-dehydrogenase (NADP+) activity [GO:0047903] (molecular function) Definition: Catalysis of the reaction: D-fructose + NADP+ = 5-dehydro-D-fructose + NADPH. Also known as: 5-keto-D-fructose reductase (NADP+), 5-ketofructose reductase (NADP(+)) activity, 5-ketofructose reductase (NADP), 5-ketofructose reductase (NADP+) activity, D-(-)fructose:(NADP+) 5-oxidoreductase activity, D-fructose:NADP+ 5-oxidoreductase activity, fructose 5-(nicotinamide adenine dinucleotide phosphate) dehydrogenase activity Sources: EC:1.1.1.124, MetaCyc:FRUCTOSE-5-DEHYDROGENASE-NADP+-RXN Relationships: is a type of oxidoreductase activity, acting on the CH-OH group of donors, NAD or NADP as acceptor [GO:0016616]